flavonoid 3'-monooxygenase activity [GO:0016711] (molecular function) Relationships: is a type of GO:0016709 Sources: EC:1.14.14.82 Also known as: NADPH:flavonoid-3'-hydroxylase activity, flavonoid 3'-hydroxylase activity, flavonoid 3-hydroxylase, flavonoid 3-monooxygenase, flavonoid,NADPH:oxygen oxidoreductase (3'-hydroxylating) Definition: Catalysis of the reaction: a flavonoid + NADPH + H+ + O2 = 3'-hydroxyflavonoid + NADP+ + H2O.